hypothalamus cell differentiation [GO:0021979] (biological process) Subtypes: hypothalamus gonadotrophin-releasing hormone neuron differentiation [GO:0021886] Sources: GOC:cls, GOC:dgh, GOC:dph, GOC:jid, GOC:mgi_curators Relationships: is a type of GO:0030154; is part of GO:0021854 Definition: The differentiation of cells that will contribute to the structure and function of the hypothalamus.